adenylate cyclase activator activity [GO:0010856] (molecular function) Sources: GOC:dph, GOC:tb Definition: Binds to and increases the activity of adenylate cyclase. Relationships: is a type of cyclase activator activity [GO:0010853]; is a type of adenylate cyclase regulator activity [GO:0010854]; positively regulates GO:0004016